{
  "gene_symbol": "EIF4G2",
  "term_label": "translation initiation factor activity",
  "gene_name": "Eukaryotic translation initiation factor 4 gamma 2",
  "gene": "UniProtKB:P78344",
  "term_id": "GO:0003743"
}